{
  "gene_name": "Calnexin",
  "gene": "UniProtKB:P27824",
  "term_label": "ERAD pathway",
  "term_id": "GO:0036503",
  "gene_symbol": "CANX"
}